dorsal vessel aortic cell fate commitment [GO:0035052] (biological process) References: PMID:12397110 Sources: GOC:bf, GOC:mtg_sensu Definition: The commitment of dorsal vessel cardioblast cells to an aortic cell fate and their capacity to differentiate into aortic cells. An example of this process is found in Drosophila melanogaster. Relationships: is a type of cell fate commitment involved in pattern specification [GO:0060581]; is a type of cardiac cell fate commitment [GO:0060911]; is part of embryonic heart tube anterior/posterior pattern specification [GO:0035054]